regulation of growth hormone receptor signaling pathway [GO:0060398] (biological process) Subtypes: GO:0060399, negative regulation of growth hormone receptor signaling pathway [GO:0060400] Also known as: regulation of growth hormone receptor signalling pathway Definition: Any process that modulates the rate, frequency or extent of the growth hormone receptor signaling pathway. The growth hormone receptor signaling pathway is the series of molecular signals generated as a consequence of growth hormone receptor binding to its physiological ligand. Sources: GOC:BHF, GOC:dph Relationships: is a type of regulation of signal transduction [GO:0009966]; regulates growth hormone receptor signaling pathway [GO:0060396]